regulation of lipophagy [GO:1904502] (biological process) Subtypes: negative regulation of lipophagy [GO:1904503], positive regulation of lipophagy [GO:1904504] Relationships: is a type of GO:0016241; regulates lipophagy [GO:0061724] Definition: Any process that modulates the frequency, rate or extent of lipophagy. References: PMID:25383539 Sources: GOC:TermGenie, GOC:autophagy, GOC:dph, GO_REF:0000058